{
  "term_label": "Unknown cellular component",
  "gene": "UniProtKB:Q5TAA0",
  "gene_name": "Tetratricopeptide repeat protein 22",
  "gene_symbol": "TTC22",
  "term_id": "UNKNOWN:0003"
}